{
  "term_id": "GO:0046961",
  "gene_name": "V-type proton ATPase subunit D",
  "gene_symbol": "ATP6V1D",
  "term_label": "proton-transporting ATPase activity, rotational mechanism",
  "gene": "UniProtKB:Q9Y5K8"
}